{
  "gene": "UniProtKB:P48167",
  "gene_name": "Glycine receptor subunit beta",
  "gene_symbol": "GLRB",
  "term_id": "GO:0060012",
  "term_label": "synaptic transmission, glycinergic"
}